{
  "term_id": "GO:0016064",
  "gene_symbol": "IGHV5-51",
  "gene": "UniProtKB:A0A0C4DH38",
  "term_label": "immunoglobulin mediated immune response",
  "gene_name": "Immunoglobulin heavy variable 5-51"
}